{
  "term_label": "plasma membrane",
  "term_id": "GO:0005886",
  "gene_name": "Dedicator of cytokinesis protein 5",
  "gene_symbol": "DOCK5",
  "gene": "UniProtKB:Q9H7D0"
}